{
  "term_id": "GO:0007417",
  "gene": "UniProtKB:P06396",
  "gene_name": "Gelsolin",
  "gene_symbol": "GSN",
  "term_label": "central nervous system development"
}